{
  "term_id": "GO:0005634",
  "gene": "UniProtKB:Q9Y6M4",
  "term_label": "nucleus",
  "gene_name": "Casein kinase I isoform gamma-3",
  "gene_symbol": "CSNK1G3"
}